GTP-dependent protein binding [GO:0030742] (MF) Relationships: is_a protein binding [GO:0005515] Definition: Binding to a protein or protein complex when at least one of the interacting partners is in the GTP-bound state. Note: This term may be used to annotate both partners in a GTP-dependent binding interaction, both the GTP-bound protein and the protein(s) which interact with it. Sources: GOC:go_curators, GOC:krc